negative regulation of protein localization to nucleolus [GO:1904750] (biological process) Definition: Any process that stops, prevents or reduces the frequency, rate or extent of protein localization to nucleolus. References: PMID:24415760 Sources: GOC:BHF, GOC:BHF_telomere, GOC:TermGenie, GOC:nc, GO_REF:0000058 Also known as: down regulation of protein localisation in nucleolus, down regulation of protein localisation to nucleolus, down regulation of protein localization in nucleolus, down regulation of protein localization to nucleolus, down-regulation of protein localisation in nucleolus, down-regulation of protein localisation to nucleolus, down-regulation of protein localization in nucleolus, down-regulation of protein localization to nucleolus, downregulation of protein localisation in nucleolus, downregulation of protein localisation to nucleolus, downregulation of protein localization in nucleolus, downregulation of protein localization to nucleolus, negative regulation of protein localisation in nucleolus, negative regulation of protein localisation to nucleolus, negative regulation of protein localization in nucleolus, inhibition of protein localisation in nucleolus, inhibition of protein localisation to nucleolus, inhibition of protein localization in nucleolus, inhibition of protein localization to nucleolus Relationships: is a type of negative regulation of protein localization to nucleus [GO:1900181]; is a type of regulation of protein localization to nucleolus [GO:1904749]; negatively regulates protein localization to nucleolus [GO:1902570]